{
  "gene_name": "Cyclin-G1",
  "gene_symbol": "CCNG1",
  "gene": "UniProtKB:P51959",
  "term_id": "GO:0000307",
  "term_label": "cyclin-dependent protein kinase holoenzyme complex"
}